{
  "term_id": "GO:0097104",
  "term_label": "postsynaptic membrane assembly",
  "gene_symbol": "NLGN3",
  "gene_name": "Neuroligin-3",
  "gene": "UniProtKB:Q9NZ94"
}